{
  "gene": "UniProtKB:Q7Z5P4",
  "term_id": "GO:0016229",
  "gene_symbol": "HSD17B13",
  "gene_name": "17-beta-hydroxysteroid dehydrogenase 13",
  "term_label": "steroid dehydrogenase activity"
}